IRES-mediated translation initiation factor activity [GO:0160297] (molecular function) Definition: A translation initiation factor activity that enables interaction with internal ribosome entry sites (IRESs) located within mRNA, promoting ribosome recruitment and assembly at internal initiation sites and translation initiation independent of the 5' cap structure. References: PMID:21118130, PMID:31913484 Relationships: is a type of translation initiation factor activity [GO:0003743]